{
  "term_label": "actomyosin structure organization",
  "gene_symbol": "EPB41L5",
  "term_id": "GO:0031032",
  "gene": "UniProtKB:Q9HCM4",
  "gene_name": "Band 4.1-like protein 5"
}